{
  "term_label": "prenylcysteine oxidase activity",
  "gene_name": "Prenylcysteine oxidase 1",
  "term_id": "GO:0001735",
  "gene_symbol": "PCYOX1",
  "gene": "UniProtKB:Q9UHG3"
}